{
  "gene_symbol": "GOLGA5",
  "gene_name": "Golgin subfamily A member 5",
  "term_id": "GO:0000301",
  "term_label": "retrograde transport, vesicle recycling within Golgi",
  "gene": "UniProtKB:Q8TBA6"
}